RIG-I binding [GO:0039552] (molecular function) Definition: Binding to RIG-I, a cytosolic pattern recognition receptor that initiates an antiviral signaling pathway upon binding to viral RNA. References: PMID:21233210 Sources: GOC:bf Also known as: DDX58 binding, DDX58/RIG-I binding Relationships: is a type of GO:0005102